{
  "gene": "UniProtKB:Q6UX65",
  "term_id": "UNKNOWN:0001",
  "gene_symbol": "DRAM2",
  "term_label": "Unknown molecular function",
  "gene_name": "DNA damage-regulated autophagy modulator protein 2"
}